{
  "gene_symbol": "ZNF266",
  "term_label": "RNA polymerase II transcription regulatory region sequence-specific DNA binding",
  "gene": "UniProtKB:Q14584",
  "gene_name": "Zinc finger protein 266",
  "term_id": "GO:0000977"
}